{
  "gene": "UniProtKB:Q96G61",
  "gene_symbol": "NUDT11",
  "term_id": "GO:0071543",
  "gene_name": "Diphosphoinositol polyphosphate phosphohydrolase 3-beta",
  "term_label": "diphosphoinositol polyphosphate metabolic process"
}